{
  "term_id": "UNKNOWN:0002",
  "term_label": "Unknown biological process",
  "gene_name": "Putative uncharacterized protein PRO0628",
  "gene": "UniProtKB:Q9UI54",
  "gene_symbol": "PRO0628"
}